regulation of bacterial-type flagellum-dependent cell motility [GO:1902021] (biological process) Also known as: regulation of bacterial-type flagellum cell motility, regulation of flagellin-based flagellar cell motility, regulation of bacterial-type flagellar cell motility Relationships: is a type of regulation of cell motility [GO:2000145]; regulates bacterial-type flagellum-dependent cell motility [GO:0071973] Sources: GOC:TermGenie, GOC:cilia, GOC:jl Definition: Any process that modulates the frequency, rate or extent of bacterial-type flagellum-dependent cell motility. Subtypes: GO:0071945, GO:1902201